negative regulation of sporangium germination [GO:0075225] (biological process) Sources: GOC:pamgo_curators Also known as: negative regulation of sporangium germination on or near host Relationships: is a type of regulation of sporangium germination [GO:0075223]; is a type of negative regulation of sporangium development [GO:0075312]; negatively regulates sporangium germination [GO:0075222] Definition: Any process that stops, prevents, or reduces the frequency, rate or extent of sporangium germination.